{
  "gene_name": "Intermediate filament family orphan 2",
  "term_id": "UNKNOWN:0002",
  "gene_symbol": "IFFO2",
  "term_label": "Unknown biological process",
  "gene": "UniProtKB:Q5TF58"
}